{
  "term_id": "GO:0015485",
  "term_label": "cholesterol binding",
  "gene": "UniProtKB:P11597",
  "gene_name": "Cholesteryl ester transfer protein",
  "gene_symbol": "CETP"
}